{
  "gene_symbol": "SORL1",
  "term_label": "post-Golgi vesicle-mediated transport",
  "gene": "UniProtKB:Q92673",
  "gene_name": "Sortilin-related receptor",
  "term_id": "GO:0006892"
}